{
  "gene": "UniProtKB:Q96LA5",
  "term_label": "immune response",
  "gene_name": "Fc receptor-like protein 2",
  "gene_symbol": "FCRL2",
  "term_id": "GO:0006955"
}